nucleosome assembly [GO:0006334] (biological process) Regulation: positively regulated by positive regulation of nucleosome disassembly [GO:0140887] Also known as: nucleosome modeling, histone chaperone Definition: The aggregation, arrangement and bonding together of a nucleosome, the beadlike structural units of eukaryotic chromatin composed of histones and DNA. Relationships: is a type of GO:0034728; is a type of protein-DNA complex assembly [GO:0065004]; is part of GO:0006325 Sources: GOC:mah